renal D-glucose absorption [GO:0035623] (biological process) Also known as: glucose reabsorption, nephron glucose absorption, renal glucose absorption Relationships: is a type of renal absorption [GO:0070293]; is a type of D-glucose transmembrane transport [GO:1904659] References: PMID:11269503 Sources: GOC:yaf Definition: A renal system process in which D-glucose is taken up from the collecting ducts and proximal and distal loops of the nephron. In non-mammalian species, absorption may occur in related structures.